neural fold folding [GO:0021505] (biological process) References: PMID:13679871, PMID:15806586 Sources: GOC:cls, GOC:dgh, GOC:dph, GOC:jid, GO_REF:0000021 Relationships: is a type of embryonic morphogenesis [GO:0048598]; is a type of morphogenesis of an epithelial fold [GO:0060571]; is part of neural fold bending [GO:0021503] Definition: The process of folding the neuroepithelium around the medial hinge point to create the neural elevations, and around the lateral hinge points to produce convergence of the folds.